{
  "gene": "UniProtKB:Q96QT6",
  "term_id": "GO:0003714",
  "gene_name": "PHD finger protein 12",
  "gene_symbol": "PHF12",
  "term_label": "transcription corepressor activity"
}